{
  "gene": "UniProtKB:Q8WV15",
  "term_label": "Unknown cellular component",
  "term_id": "UNKNOWN:0003",
  "gene_symbol": "TMEM255B",
  "gene_name": "Transmembrane protein 255B"
}